{
  "gene_symbol": "TGFBR3",
  "term_label": "transforming growth factor beta receptor signaling pathway",
  "gene_name": "Transforming growth factor beta receptor type 3",
  "gene": "UniProtKB:Q03167",
  "term_id": "GO:0007179"
}